{
  "gene_name": "Diphosphoinositol polyphosphate phosphohydrolase 2",
  "term_label": "nucleus",
  "term_id": "GO:0005634",
  "gene_symbol": "NUDT4",
  "gene": "UniProtKB:Q9NZJ9"
}